{
  "gene_name": "Prolyl endopeptidase-like",
  "gene_symbol": "PREPL",
  "term_id": "GO:0005856",
  "term_label": "cytoskeleton",
  "gene": "UniProtKB:Q4J6C6"
}